muscle tissue morphogenesis [GO:0060415] (biological process) Subtypes: GO:0003150, cardiac muscle tissue morphogenesis [GO:0055008], GO:0060414 Relationships: is a type of tissue morphogenesis [GO:0048729]; is part of muscle organ morphogenesis [GO:0048644] Definition: The process in which the anatomical structures of muscle tissue are generated and organized. Muscle tissue consists of a set of cells that are part of an organ and carry out a contractive function. Sources: GOC:dph